{
  "term_id": "GO:0005634",
  "gene_name": "Coiled-coil and C2 domain-containing protein 1A",
  "gene_symbol": "CC2D1A",
  "term_label": "nucleus",
  "gene": "UniProtKB:Q6P1N0"
}